{
  "gene_symbol": "LTK",
  "term_id": "GO:0045664",
  "term_label": "regulation of neuron differentiation",
  "gene_name": "Leukocyte tyrosine kinase receptor",
  "gene": "UniProtKB:P29376"
}